ATP:ATP adenylyltransferase activity [GO:0141192] (molecular function) Definition: Catalysis of the reaction: 2 ATP + H+ = diphosphate + P(1),P(4)-bis(5'-adenosyl)tetraphosphate. References: PMID:16884494, PMID:19710017, PMID:27398309 Sources: RHEA:34935 Also known as: adenine triphosphate adenylyltransferase activity Relationships: is a type of adenylyltransferase activity [GO:0070566]